R7 cell fate commitment [GO:0007465] (biological process) References: PMID:3076112, PMID:3937883 Relationships: is a type of compound eye photoreceptor fate commitment [GO:0001752]; is part of R7 cell differentiation [GO:0045466] Regulation: regulated by regulation of R7 cell fate commitment [GO:0106396]; positively regulated by positive regulation of R7 cell fate commitment [GO:0106397]; negatively regulated by negative regulation of R7 cell fate commitment [GO:0106398] Definition: The process in which the R7 photoreceptor commits to its cell fate. The R7 receptor contributes the central part of the rhabdomere in the apical parts of the ommatidium.